transmitting tissue development [GO:0010500] (biological process) Definition: The process whose specific outcome is the progression of the transmitting tract over time, from its formation to the mature structure. The transmitting tissue is the tissue in the style of a carpel through which the pollen tube grows; it connects the stigma and the inside of ovary. Relationships: is a type of gynoecium development [GO:0048467] References: PMID:17855426